floral organ senescence [GO:0080187] (biological process) Relationships: is a type of plant organ senescence [GO:0090693]; is part of floral organ development [GO:0048437] Definition: The last stage of flower development during which programmed degradation of macromolecules and nutrient recycling take place. References: PMID:19380421, PMID:21689171 Note: Includes senescence of petals, sepals, anthers, and any other plant organ that is part of a flower. Floral organ senescence may follow pollination. In some flowers, the organs of the corolla abscise before they senesce.